{
  "gene": "UniProtKB:Q9H1E5",
  "gene_symbol": "TMX4",
  "term_id": "GO:0012505",
  "gene_name": "Thioredoxin-related transmembrane protein 4",
  "term_label": "endomembrane system"
}